calcitonin family receptor activity [GO:0097642] (molecular function) Subtypes: adrenomedullin receptor activity [GO:0001605], calcitonin gene-related peptide receptor activity [GO:0001635], calcitonin receptor activity [GO:0004948], GO:0097643 References: PMID:10871296, PMID:12037140, PMID:18687416 Sources: GOC:bhm, InterPro:IPR003287 Relationships: is a type of GO:0008528 Definition: Combining with any member of the calcitonin family (e.g. adrenomedullin, adrenomedullin 2 (intermedin), amylin, calcitonin and calcitonin gene-related peptides (CGRPs)) to initiate a change in cell activity.